epithelial to mesenchymal transition involved in coronary vasculature morphogenesis [GO:0003201] (biological process) Relationships: is a type of GO:0060317; is part of coronary vasculature morphogenesis [GO:0060977] Definition: A transition where a cardiac epithelial cell loses apical/basolateral polarity, severs intercellular adhesive junctions, degrades basement membrane components and becomes a migratory mesenchymal cell that will contribute to the shaping of the coronary vasculature. Sources: GOC:mtg_heart